{
  "term_id": "GO:0003729",
  "gene_symbol": "DDX43",
  "gene": "UniProtKB:Q9NXZ2",
  "gene_name": "Probable ATP-dependent RNA helicase DDX43",
  "term_label": "mRNA binding"
}